{
  "gene_name": "Acyl-coenzyme A synthetase ACSM2B, mitochondrial",
  "gene_symbol": "ACSM2B",
  "term_id": "GO:0006637",
  "term_label": "acyl-CoA metabolic process",
  "gene": "UniProtKB:Q68CK6"
}